dolichol O-acyltransferase activity [GO:0047872] (molecular function) Also known as: acyl-CoA:dolichol acyltransferase activity, palmitoyl-CoA:dolichol O-palmitoyltransferase activity Sources: EC:2.3.1.123, MetaCyc:DOLICHOL-O-ACYLTRANSFERASE-RXN Relationships: is a type of O-acyltransferase activity [GO:0008374] Definition: Catalysis of the reaction: palmitoyl-CoA + dolichol = CoA + dolichyl palmitate.